{
  "term_id": "GO:0016038",
  "term_label": "absorption of visible light",
  "gene_name": "Long-wave-sensitive opsin 1",
  "gene_symbol": "OPN1LW",
  "gene": "UniProtKB:P04000"
}